{
  "term_label": "cytoplasm",
  "gene": "UniProtKB:Q15773",
  "gene_name": "Myeloid leukemia factor 2",
  "gene_symbol": "MLF2",
  "term_id": "GO:0005737"
}